{
  "term_label": "cysteine-type deubiquitinase activity",
  "gene": "UniProtKB:Q14694",
  "gene_name": "Ubiquitin carboxyl-terminal hydrolase 10",
  "gene_symbol": "USP10",
  "term_id": "GO:0004843"
}